{
  "gene_name": "Zinc finger protein 554",
  "gene_symbol": "ZNF554",
  "term_label": "RNA polymerase II transcription regulatory region sequence-specific DNA binding",
  "term_id": "GO:0000977",
  "gene": "UniProtKB:Q86TJ5"
}